{
  "gene_name": "Rho GTPase-activating protein 15",
  "term_label": "plasma membrane",
  "gene": "UniProtKB:Q53QZ3",
  "gene_symbol": "ARHGAP15",
  "term_id": "GO:0005886"
}